{
  "term_label": "plasma membrane",
  "term_id": "GO:0005886",
  "gene_name": "Olfactory receptor 2Z1",
  "gene": "UniProtKB:Q8NG97",
  "gene_symbol": "OR2Z1"
}